{
  "gene_name": "5-hydroxytryptamine receptor 3B",
  "term_id": "GO:0022850",
  "term_label": "serotonin-gated monoatomic cation channel activity",
  "gene_symbol": "HTR3B",
  "gene": "UniProtKB:O95264"
}